{
  "term_id": "UNKNOWN:0002",
  "term_label": "Unknown biological process",
  "gene": "UniProtKB:Q6ZTU2",
  "gene_symbol": "EP400P1",
  "gene_name": "Putative EP400-like protein"
}